{
  "term_label": "plasminogen activation",
  "gene_name": "Urokinase-type plasminogen activator",
  "gene_symbol": "PLAU",
  "gene": "UniProtKB:P00749",
  "term_id": "GO:0031639"
}